{
  "gene_name": "Cilia- and flagella-associated protein 69",
  "gene_symbol": "CFAP69",
  "term_id": "GO:0097730",
  "gene": "UniProtKB:A5D8W1",
  "term_label": "non-motile cilium"
}